positive regulation of heme biosynthetic process [GO:0070455] (biological process) Sources: GOC:mah Also known as: positive regulation of haem biosynthetic process, positive regulation of heme anabolism, positive regulation of heme biosynthesis, positive regulation of heme formation, positive regulation of heme synthesis, up regulation of heme biosynthetic process, up-regulation of heme biosynthetic process, upregulation of heme biosynthetic process, activation of heme biosynthetic process, stimulation of heme biosynthetic process Relationships: is a type of GO:0070453; is_a positive regulation of tetrapyrrole biosynthetic process [GO:1901465]; positively regulates heme biosynthetic process [GO:0006783] Definition: Any process that activates or increases the frequency, rate or extent of the chemical reactions and pathways resulting in the formation of heme.